{
  "gene": "UniProtKB:Q86Y91",
  "term_id": "GO:0016887",
  "term_label": "ATP hydrolysis activity",
  "gene_name": "Kinesin-like protein KIF18B",
  "gene_symbol": "KIF18B"
}